{
  "gene_symbol": "SEPTIN1",
  "gene_name": "Septin-1",
  "term_label": "microtubule cytoskeleton",
  "gene": "UniProtKB:Q8WYJ6",
  "term_id": "GO:0015630"
}